{
  "term_id": "GO:0005634",
  "gene_name": "WD repeat-containing protein 70",
  "gene_symbol": "WDR70",
  "term_label": "nucleus",
  "gene": "UniProtKB:Q9NW82"
}